{
  "gene_symbol": "RANBP17",
  "gene_name": "Ran-binding protein 17",
  "term_label": "cytoplasm",
  "term_id": "GO:0005737",
  "gene": "UniProtKB:Q9H2T7"
}